{
  "gene_symbol": "INSM1",
  "term_label": "negative regulation of transcription by RNA polymerase II",
  "term_id": "GO:0000122",
  "gene": "UniProtKB:Q01101",
  "gene_name": "Insulinoma-associated protein 1"
}